{
  "gene": "UniProtKB:P18505",
  "gene_name": "Gamma-aminobutyric acid receptor subunit beta-1",
  "term_label": "chloride channel activity",
  "term_id": "GO:0005254",
  "gene_symbol": "GABRB1"
}